{
  "gene": "UniProtKB:P41236",
  "term_label": "intracellular signal transduction",
  "gene_name": "Protein phosphatase inhibitor 2",
  "term_id": "GO:0035556",
  "gene_symbol": "PPP1R2"
}